{
  "gene": "UniProtKB:Q8WXE9",
  "term_label": "AP-2 adaptor complex",
  "gene_name": "Stonin-2",
  "term_id": "GO:0030122",
  "gene_symbol": "STON2"
}